{
  "term_label": "apical plasma membrane",
  "gene_symbol": "ABCB4",
  "gene_name": "Phosphatidylcholine translocator ABCB4",
  "term_id": "GO:0016324",
  "gene": "UniProtKB:P21439"
}